{
  "term_label": "postsynaptic density",
  "gene_name": "Nitric oxide synthase 1",
  "term_id": "GO:0014069",
  "gene": "UniProtKB:P29475",
  "gene_symbol": "NOS1"
}